{
  "term_id": "GO:1905668",
  "gene_name": "Alpha_beta hydrolase domain-containing protein 17A",
  "gene": "UniProtKB:Q96GS6",
  "gene_symbol": "ABHD17A",
  "term_label": "positive regulation of protein localization to endosome"
}